{
  "gene_name": "Glycerol-3-phosphate dehydrogenase, mitochondrial",
  "term_label": "mitochondrion",
  "term_id": "GO:0005739",
  "gene": "UniProtKB:P43304",
  "gene_symbol": "GPD2"
}